{
  "term_label": "positive regulation of protein ubiquitination",
  "gene": "UniProtKB:Q3KP66",
  "gene_name": "Innate immunity activator protein",
  "term_id": "GO:0031398",
  "gene_symbol": "INAVA"
}